adherens junction assembly [GO:0034333] (biological process) Definition: The aggregation, arrangement and bonding together of a set of components to form an adherens junction. An adherens junction is a cell-cell junction composed of the epithelial cadherin-catenin complex at which the cytoplasmic face of the plasma membrane is attached to actin filaments. Sources: GOC:aruk, GOC:bc, GOC:mah Also known as: adherens junction formation Relationships: is a type of cell-cell junction assembly [GO:0007043]; is a type of adherens junction organization [GO:0034332] Subtypes: nephrocyte diaphragm assembly [GO:0036059], zonula adherens assembly [GO:0045186]